intestinal lipid catabolic process [GO:0044258] (biological process) Definition: The chemical reactions and pathways resulting in the breakdown into fatty acids and monoglycerides of lipids in the small intestine. Lipids are broken down by lipases released by the pancreas. References: PMID:7018485 Sources: GOC:jl Also known as: intestinal lipid breakdown, intestinal lipid catabolism, intestinal lipid degradation Relationships: is a type of GO:0016042